{
  "gene_name": "Zinc finger protein 891",
  "gene_symbol": "ZNF891",
  "term_label": "nucleus",
  "gene": "UniProtKB:A8MT65",
  "term_id": "GO:0005634"
}